{
  "gene_symbol": "GZMB",
  "gene": "UniProtKB:P10144",
  "term_id": "GO:0140507",
  "term_label": "granzyme-mediated programmed cell death signaling pathway",
  "gene_name": "Granzyme B"
}